asperthecin metabolic process [GO:0036182] (biological process) Definition: The chemical reactions and pathways involving asperthecin, an anthraquinone pigment obtained from the mould Aspergillus nidulans. Sources: GOC:di Also known as: asperthecin metabolism Relationships: is a type of GO:0018958; is a type of GO:0019748; is a type of ketone metabolic process [GO:0042180] Subtypes: asperthecin catabolic process [GO:0036183], asperthecin biosynthetic process [GO:0036184]